{
  "term_id": "GO:0010975",
  "gene_symbol": "FRMD7",
  "gene_name": "FERM domain-containing protein 7",
  "term_label": "regulation of neuron projection development",
  "gene": "UniProtKB:Q6ZUT3"
}